{
  "gene_symbol": "ARHGEF4",
  "gene_name": "Rho guanine nucleotide exchange factor 4",
  "gene": "UniProtKB:Q9NR80",
  "term_label": "Unknown biological process",
  "term_id": "UNKNOWN:0002"
}